chloride ion binding [GO:0031404] (molecular function) Sources: GOC:mah Definition: Binding to a chloride ion (Cl-). Relationships: is a type of anion binding [GO:0043168] Also known as: Cl- ion binding, chloride binding